rhombomere cell proliferation [GO:0022034] (biological process) Definition: The multiplication or reproduction of rhombomere cells, resulting in the expansion of the cell population. Sources: GOC:cls, GOC:dgh, GOC:dph, GOC:jid, GO_REF:0000021 Relationships: is a type of GO:0061351; is part of GO:0021546